{
  "gene_symbol": "CXCL13",
  "gene": "UniProtKB:O43927",
  "term_label": "inflammatory response",
  "term_id": "GO:0006954",
  "gene_name": "C-X-C motif chemokine 13"
}